{
  "term_label": "positive regulation of synaptic transmission",
  "term_id": "GO:0050806",
  "gene_name": "Calsyntenin-3",
  "gene": "UniProtKB:Q9BQT9",
  "gene_symbol": "CLSTN3"
}